{
  "gene_name": "Arf-GAP with SH3 domain, ANK repeat and PH domain-containing protein 1",
  "term_label": "podosome",
  "gene_symbol": "ASAP1",
  "gene": "UniProtKB:Q9ULH1",
  "term_id": "GO:0002102"
}